L-valine catabolic process [GO:0006574] (biological process) Subtypes: GO:1902697 Definition: The chemical reactions and pathways resulting in the breakdown of L-valine, 2-amino-3-methylbutanoic acid. Relationships: is a type of valine metabolic process [GO:0006573]; is a type of branched-chain amino acid catabolic process [GO:0009083]; is a type of L-amino acid catabolic process [GO:0170035]; is a type of proteinogenic amino acid catabolic process [GO:0170040] Sources: GOC:ai Also known as: valine breakdown, valine catabolism, valine degradation